{
  "term_id": "GO:0051233",
  "gene_name": "Microtubule-associated protein RP_EB family member 1",
  "gene": "UniProtKB:Q15691",
  "gene_symbol": "MAPRE1",
  "term_label": "spindle midzone"
}